{
  "gene_name": "Gametogenetin",
  "gene_symbol": "GGN",
  "term_label": "Unknown cellular component",
  "term_id": "UNKNOWN:0003",
  "gene": "UniProtKB:Q86UU5"
}